core promoter sequence-specific DNA binding [GO:0001046] (molecular function) Subtypes: RNA polymerase II core promoter sequence-specific DNA binding [GO:0000979], RNA polymerase I core promoter sequence-specific DNA binding [GO:0001164] Relationships: is a type of transcription cis-regulatory region binding [GO:0000976] Definition: Binding to a sequence of DNA that is part of a core promoter region. The core promoter is composed of the transcription start site and binding sites for the RNA polymerase and the basal transcription machinery. The transcribed region might be described as a gene, cistron, or operon. Regulation: negatively regulated by negative regulation of core promoter binding [GO:1904797]; positively regulated by positive regulation of core promoter binding [GO:1904798] Sources: GOC:pg, GOC:txnOH Also known as: bacterial-type RNA polymerase core promoter sequence-specific DNA binding, eubacterial-type RNA polymerase core promoter sequence-specific DNA binding, core promoter binding